regulation of mini excitatory postsynaptic potential [GO:0061884] (biological process) References: PMID:20395454 Sources: GOC:aruk, GOC:bc Definition: Any process that modulates the frequency, rate or extent of mini excitatory postsynaptic potential. Mini excitatory postsynaptic potential is a process that leads to a temporary increase in postsynaptic potential due to the flow of positively charged ions into the postsynaptic cell, induced by the spontaneous release of a single vesicle of an excitatory neurotransmitter into the synapse. Relationships: is a type of modulation of excitatory postsynaptic potential [GO:0098815]; regulates mini excitatory postsynaptic potential [GO:0098816] Subtypes: positive regulation of mini excitatory postsynaptic potential [GO:0061885], negative regulation of mini excitatory postsynaptic potential [GO:0061886]